hydroxylysine biosynthetic process [GO:0046947] (biological process) Sources: ISBN:0198506732 Relationships: is a type of GO:0009067; is a type of GO:0042398; is a type of GO:0170043 Also known as: hydroxylysine anabolism, hydroxylysine biosynthesis, hydroxylysine formation, hydroxylysine synthesis Definition: The chemical reactions and pathways resulting in the formation of hydroxylysine (5-hydroxy-2,6-diaminohexanoic acid), a chiral alpha-amino acid.